Toll signaling pathway [GO:0008063] (biological process) Definition: The series of molecular signals initiated by an extracellular ligand binding to the receptor Toll on the surface of a target cell, and ending with the regulation of a downstream cellular process, e.g. transcription. References: PMID:11135568, PMID:19126860 Sources: GOC:go_curators Relationships: is a type of cell surface receptor signaling pathway [GO:0007166] Regulation: regulated by GO:0008592; negatively regulated by negative regulation of Toll signaling pathway [GO:0045751]; positively regulated by positive regulation of Toll signaling pathway [GO:0045752] Also known as: Tl signaling pathway, Tl signalling pathway, Toll signalling pathway